{
  "gene_name": "Glycerophosphocholine phosphodiesterase GPCPD1",
  "gene": "UniProtKB:Q9NPB8",
  "term_id": "GO:0046475",
  "gene_symbol": "GPCPD1",
  "term_label": "glycerophospholipid catabolic process"
}